positive regulation of amine catabolic process [GO:0033243] (biological process) Definition: Any process that activates or increases the frequency, rate or extent of the chemical reactions and pathways leading to the breakdown of amines. Sources: GOC:mah Also known as: positive regulation of amine breakdown, positive regulation of amine catabolism, positive regulation of amine degradation Relationships: is a type of positive regulation of catabolic process [GO:0009896]; is a type of GO:0033240; is a type of regulation of amine catabolic process [GO:0033241]; positively regulates GO:0009310